{
  "term_id": "GO:0007268",
  "gene_symbol": "CACNB2",
  "gene": "UniProtKB:Q08289",
  "term_label": "chemical synaptic transmission",
  "gene_name": "Voltage-dependent L-type calcium channel subunit beta-2"
}